{
  "gene_name": "Cytoplasmic protein NCK2",
  "gene_symbol": "NCK2",
  "gene": "UniProtKB:O43639",
  "term_id": "GO:0030971",
  "term_label": "receptor tyrosine kinase binding"
}